{
  "gene": "UniProtKB:P10826",
  "gene_name": "Retinoic acid receptor beta",
  "term_id": "GO:0048384",
  "term_label": "retinoic acid receptor signaling pathway",
  "gene_symbol": "RARB"
}